{
  "term_label": "chromatin binding",
  "gene": "UniProtKB:Q99549",
  "gene_name": "M-phase phosphoprotein 8",
  "term_id": "GO:0003682",
  "gene_symbol": "MPHOSPH8"
}